{
  "term_id": "GO:0007043",
  "gene": "UniProtKB:Q8IXH8",
  "term_label": "cell-cell junction assembly",
  "gene_symbol": "CDH26",
  "gene_name": "Cadherin-like protein 26"
}